{
  "gene_symbol": "LIMA1",
  "gene_name": "LIM domain and actin-binding protein 1",
  "gene": "UniProtKB:Q9UHB6",
  "term_label": "actin cytoskeleton",
  "term_id": "GO:0015629"
}